IgW immunoglobulin complex [GO:0071758] (cellular component) Note: Note that an IgW immunoglobulin complex has the function of antigen binding if a suitable antigen is available. Note that IgW is found in fish. Sources: GOC:add, ISBN:0781765196 Definition: A protein complex composed of two identical immunoglobulin heavy chains of the IgW isotype and two identical immunoglobulin light chains, held together by disulfide bonds. An IgW immunoglobulin complex may be embedded in the plasma membrane or present in the extracellular space, in mucosal areas or other tissues, or circulating in the blood or lymph. Relationships: is a type of GO:0019814